{
  "term_label": "Unknown molecular function",
  "gene": "UniProtKB:Q86VQ1",
  "gene_name": "Glucocorticoid-induced transcript 1 protein",
  "gene_symbol": "GLCCI1",
  "term_id": "UNKNOWN:0001"
}